store-operated calcium entry [GO:0002115] (biological process) Relationships: is_a GO:0006816 Regulation: negatively regulated by negative regulation of store-operated calcium entry [GO:0106128]; positively regulated by positive regulation of store-operated calcium entry [GO:0106129]; regulated by regulation of store-operated calcium entry [GO:2001256] References: PMID:11120592, PMID:17956991 Sources: GOC:hjd Also known as: calcium ion import, SOCE, capacitative calcium entry, store-operated calcium import Note: SOCE is initiated by response to stiumlation of membrane receptors leading to the hydrolysis ofphosphatidylinositol bisphosphate (PIP2), inositol 1,4,5-trisphosphate (IP3) generation, and IP3-mediated calcium ion release from the endoplasmic reticulum. Definition: A calcium ion entry mechanism in the plasma membrane activated by the depletion of calcium ion from the internal calcium ion store in the endoplasmic reticulum.